{
  "gene_symbol": "RAC2",
  "gene": "UniProtKB:P15153",
  "term_id": "GO:0008360",
  "term_label": "regulation of cell shape",
  "gene_name": "Ras-related C3 botulinum toxin substrate 2"
}